{
  "term_label": "Unknown molecular function",
  "gene": "UniProtKB:Q13938",
  "gene_name": "Calcyphosin",
  "term_id": "UNKNOWN:0001",
  "gene_symbol": "CAPS"
}